cross bridge cycling involved in regulation of the velocity of shortening in skeletal muscle contraction [GO:0014868] (biological process) Sources: GOC:mtg_muscle Relationships: is a type of regulation of muscle filament sliding involved in regulation of the velocity of shortening in skeletal muscle contraction [GO:0014880] Definition: A process in which cross bridges are broken and reformed during filament sliding as part of the regulation of the velocity of shortening in skeletal muscle contraction.